{
  "gene_name": "Humanin",
  "term_id": "GO:1900118",
  "gene_symbol": "MT-RNR2",
  "gene": "UniProtKB:Q8IVG9",
  "term_label": "negative regulation of execution phase of apoptosis"
}